{
  "gene_symbol": "ABCG1",
  "gene": "UniProtKB:P45844",
  "term_label": "plasma membrane",
  "term_id": "GO:0005886",
  "gene_name": "ATP-binding cassette sub-family G member 1"
}